{
  "gene": "UniProtKB:Q9UBF9",
  "term_id": "GO:0043025",
  "gene_symbol": "MYOT",
  "gene_name": "Myotilin",
  "term_label": "neuronal cell body"
}